protein insertion into plasma membrane raft [GO:0044859] (biological process) Definition: The process in which a protein is incorporated into a plasma membrane raft. Sources: GOC:jl Relationships: is a type of GO:0071210; is a type of GO:0098737